{
  "gene_symbol": "SPATA22",
  "term_label": "regulation of meiotic cell cycle",
  "gene_name": "Spermatogenesis-associated protein 22",
  "term_id": "GO:0051445",
  "gene": "UniProtKB:Q8NHS9"
}